nitrate reductase (NADH) activity [GO:0009703] (molecular function) Sources: RHEA:17913 Also known as: assimilatory nitrate reductase activity, NADH:nitrate reductase activity, NADH-dependent nitrate reductase activity, NADH-nitrate reductase activity, NADH:nitrate oxidoreductase activity, assimilatory NADH: nitrate reductase activity, assimilatory NADH:nitrate reductase activity, nitrate reductase (NADH(2)) activity, nitrate reductase (NADH2), nitrite:NAD+ oxidoreductase activity Definition: Catalysis of the reaction: nitrite + NAD+ + H2O = nitrate + NADH + H+. Relationships: is a type of GO:0050463